regulation of auxin polar transport [GO:2000012] (biological process) Sources: GOC:obol Definition: Any process that modulates the frequency, rate or extent of auxin polar transport. Relationships: is a type of regulation of hormone levels [GO:0010817]; is a type of GO:0051049; regulates auxin polar transport [GO:0009926]